membrane repolarization during AV node cell action potential [GO:0086049] (biological process) Definition: The process in which ions are transported across a membrane such that the AV node cardiac muscle cell membrane potential changes in the direction from the positive membrane potential at the peak of the action potential towards the negative resting potential. Sources: GOC:BHF, GOC:dph, GOC:mtg_cardiac_conduct_nov11 Relationships: is a type of membrane repolarization during cardiac muscle cell action potential [GO:0086013]; is part of AV node cell action potential [GO:0086016] Also known as: membrane repolarization involved in regulation of AV node cardiac muscle cell action potential, membrane repolarization involved in regulation of atrioventricular node cardiac muscle cell action potential